{
  "gene_name": "POU domain, class 3, transcription factor 2",
  "gene": "UniProtKB:P20265",
  "term_label": "Unknown cellular component",
  "gene_symbol": "POU3F2",
  "term_id": "UNKNOWN:0003"
}